{
  "gene_symbol": "KCNS3",
  "gene": "UniProtKB:Q9BQ31",
  "term_id": "GO:0071805",
  "gene_name": "Potassium voltage-gated channel subfamily S member 3",
  "term_label": "potassium ion transmembrane transport"
}